metanephric DCT cell differentiation [GO:0072240] (biological process) Relationships: is a type of DCT cell differentiation [GO:0072069]; is a type of cell differentiation involved in metanephros development [GO:0072202]; is part of metanephric distal convoluted tubule development [GO:0072221] Regulation: regulated by GO:2000592; negatively regulated by negative regulation of metanephric DCT cell differentiation [GO:2000593]; positively regulated by GO:2000594 Definition: The process in which relatively unspecialized cells acquire specialized structural and/or functional features that characterize the distal convoluted tubule cells of the metanephros as it progresses from its formation to the mature state. Also known as: metanephric distal convoluted tubule cell differentiation Sources: GOC:mtg_kidney_jan10